positive regulation of hemopoiesis [GO:1903708] (BP) Note: An example of this is Atg7 in mouse (UniProt symbol, Q9D906) in PMID:20080761, inferred from mutant phenotype. Definition: Any process that activates or increases the frequency, rate or extent of hemopoiesis. References: PMID:20080761 Sources: GOC:PARL, GOC:TermGenie, GOC:pad, GO_REF:0000058 Also known as: positive regulation of blood cell biosynthesis, positive regulation of blood cell formation, positive regulation of haemopoiesis, positive regulation of hematopoiesis, up regulation of blood cell biosynthesis, up regulation of blood cell formation, up regulation of haemopoiesis, up regulation of hematopoiesis, up regulation of hemopoiesis, up-regulation of blood cell biosynthesis, up-regulation of blood cell formation, up-regulation of haemopoiesis, up-regulation of hematopoiesis, up-regulation of hemopoiesis, upregulation of blood cell biosynthesis, upregulation of blood cell formation, upregulation of haemopoiesis, upregulation of hematopoiesis, upregulation of hemopoiesis, activation of blood cell biosynthesis, activation of blood cell formation, activation of haemopoiesis, activation of hematopoiesis, activation of hemopoiesis Relationships: is a type of positive regulation of immune system process [GO:0002684]; is a type of positive regulation of cell development [GO:0010720]; is a type of positive regulation of multicellular organismal process [GO:0051240]; is a type of regulation of hemopoiesis [GO:1903706]; positively regulates hemopoiesis [GO:0030097] Subtypes: positive regulation of leukocyte differentiation [GO:1902107]